{
  "gene": "UniProtKB:O60814",
  "gene_name": "Histone H2B type 1-K",
  "term_label": "antibacterial humoral response",
  "term_id": "GO:0019731",
  "gene_symbol": "H2BC12"
}